{
  "gene_name": "Heterogeneous nuclear ribonucleoprotein L-like",
  "gene_symbol": "HNRNPLL",
  "term_id": "GO:0043484",
  "term_label": "regulation of RNA splicing",
  "gene": "UniProtKB:Q8WVV9"
}